{
  "gene_symbol": "DRP2",
  "term_label": "plasma membrane",
  "term_id": "GO:0005886",
  "gene": "UniProtKB:Q13474",
  "gene_name": "Dystrophin-related protein 2"
}